{
  "gene": "UniProtKB:A6NNA5",
  "term_id": "GO:0000981",
  "gene_name": "Dorsal root ganglia homeobox protein",
  "gene_symbol": "DRGX",
  "term_label": "DNA-binding transcription factor activity, RNA polymerase II-specific"
}